 [oboInOwl#is:class:level]